{
  "gene": "UniProtKB:Q96NB1",
  "term_label": "cilium assembly",
  "gene_name": "Centrosomal protein 20",
  "term_id": "GO:0060271",
  "gene_symbol": "CEP20"
}